{
  "term_label": "cytokinetic process",
  "gene": "UniProtKB:P50995",
  "gene_name": "Annexin A11",
  "gene_symbol": "ANXA11",
  "term_id": "GO:0032506"
}